{
  "term_id": "GO:1990070",
  "term_label": "TRAPPI protein complex",
  "gene": "UniProtKB:Q8IUR0",
  "gene_symbol": "TRAPPC5",
  "gene_name": "Trafficking protein particle complex subunit 5"
}